{
  "gene_name": "Receptor expression-enhancing protein 4",
  "term_label": "microtubule binding",
  "gene": "UniProtKB:Q9H6H4",
  "gene_symbol": "REEP4",
  "term_id": "GO:0008017"
}